{
  "gene_name": "CX3C chemokine receptor 1",
  "term_label": "positive regulation of cytosolic calcium ion concentration",
  "term_id": "GO:0007204",
  "gene": "UniProtKB:P49238",
  "gene_symbol": "CX3CR1"
}